plasma membrane proton-transporting V-type ATPase complex [GO:0033181] (cellular component) Also known as: plasma membrane hydrogen ion-transporting ATPase Definition: A proton-transporting two-sector ATPase complex found in the plasma membrane. Sources: GOC:mah Relationships: is a type of GO:0033176; is a type of plasma membrane protein complex [GO:0098797]